{
  "gene": "UniProtKB:Q8NGH3",
  "term_label": "detection of chemical stimulus involved in sensory perception of smell",
  "gene_name": "Olfactory receptor 2D3",
  "term_id": "GO:0050911",
  "gene_symbol": "OR2D3"
}